{
  "gene": "UniProtKB:Q13242",
  "term_label": "mRNA binding",
  "gene_symbol": "SRSF9",
  "gene_name": "Serine_arginine-rich splicing factor 9",
  "term_id": "GO:0003729"
}